{
  "term_id": "UNKNOWN:0002",
  "term_label": "Unknown biological process",
  "gene_symbol": "C2CD4D",
  "gene": "UniProtKB:B7Z1M9",
  "gene_name": "C2 calcium-dependent domain-containing protein 4D"
}